vanadium ion transport [GO:0015676] (biological process) Definition: The directed movement of vanadium (V) ions into, out of or within a cell, or between cells, by means of some agent such as a transporter or pore. Relationships: is a type of transition metal ion transport [GO:0000041] Sources: GOC:ai